NMDA selective glutamate receptor complex [GO:0017146] (cellular component) References: PMID:8294079 Definition: An assembly of four or five subunits which form a structure with an extracellular N-terminus and a large loop that together form the ligand binding domain. The C-terminus is intracellular. The ionotropic glutamate receptor complex itself acts as a ligand gated ion channel; on binding glutamate, charged ions pass through a channel in the center of the receptor complex. NMDA receptors are composed of assemblies of NR1 subunits (Figure 3) and NR2 subunits, which can be one of four separate gene products (NR2A-D). Expression of both subunits are required to form functional channels. The glutamate binding domain is formed at the junction of NR1 and NR2 subunits. NMDA receptors are permeable to calcium ions as well as being permeable to other ions. Thus NMDA receptor activation leads to a calcium influx into the post-synaptic cells, a signal thought to be crucial for the induction of NMDA-receptor dependent LTP and LTD. Relationships: is_a GO:0008328 Also known as: N-methyl-D-aspartate selective glutamate receptor complex, NMDA-selective glutamate receptor